{
  "term_label": "extracellular matrix structural constituent conferring tensile strength",
  "gene_symbol": "COL8A2",
  "gene_name": "Collagen alpha-2(VIII) chain",
  "term_id": "GO:0030020",
  "gene": "UniProtKB:P25067"
}